positive regulation of synaptic transmission [GO:0050806] (biological process) Definition: Any process that activates or increases the frequency, rate or extent of synaptic transmission, the process of communication from a neuron to a target (neuron, muscle, or secretory cell) across a synapse. Sources: GOC:ai Also known as: up regulation of synaptic transmission, up-regulation of synaptic transmission, upregulation of synaptic transmission, activation of synaptic transmission, stimulation of synaptic transmission Relationships: is a type of positive regulation of cell communication [GO:0010647]; is a type of positive regulation of signaling [GO:0023056]; is a type of modulation of chemical synaptic transmission [GO:0050804]; positively regulates chemical synaptic transmission [GO:0007268] Subtypes: positive regulation of neurotransmitter secretion [GO:0001956], GO:0032224, positive regulation of synaptic transmission, dopaminergic [GO:0032226], positive regulation of synaptic transmission, GABAergic [GO:0032230], long-term strengthening of neuromuscular junction [GO:0042062], positive regulation of synaptic transmission, glutamatergic [GO:0051968], positive regulation of synaptic transmission, glycinergic [GO:0060094], long-term synaptic potentiation [GO:0060291], GO:1900075, positive regulation of long-term synaptic potentiation [GO:1900273], GO:1900453